{
  "gene": "UniProtKB:Q63HM2",
  "gene_name": "Pecanex-like protein 4",
  "term_id": "UNKNOWN:0003",
  "term_label": "Unknown cellular component",
  "gene_symbol": "PCNX4"
}